{
  "term_label": "Unknown cellular component",
  "term_id": "UNKNOWN:0003",
  "gene_symbol": "UBE2R2",
  "gene": "UniProtKB:Q712K3",
  "gene_name": "Ubiquitin-conjugating enzyme E2 R2"
}